positive stranded viral RNA replication [GO:0039690] (biological process) Definition: A viral genome replication process where the template genome is positive stranded, single stranded RNA ((+)ssRNA). Replication of the positive strand leads to dsRNA formation, which in turn is transcribed into positive single stranded RNA. Sources: GOC:bf, GOC:jl, VZ:1116 Also known as: ss(+) viral RNA replication Relationships: is_a viral RNA genome replication [GO:0039694]